negative regulation of chromatin organization [GO:1905268] (BP) References: PMID:654321 Sources: GOC:TermGenie, GOC:pr, GOC:vw, GO_REF:0000058 Subtypes: negative regulation of heterochromatin formation [GO:0031452], GO:0120262, negative regulation of chromatin looping [GO:0160164], negative regulation of transcription initiation-coupled chromatin remodeling [GO:0160217] Relationships: is a type of negative regulation of cellular component organization [GO:0051129]; is a type of regulation of chromatin organization [GO:1902275]; negatively regulates chromatin organization [GO:0006325] Also known as: down regulation of chromatin organisation, down regulation of chromatin organization, down regulation of establishment or maintenance of chromatin architecture, down-regulation of chromatin organisation, down-regulation of chromatin organization, down-regulation of establishment or maintenance of chromatin architecture, downregulation of chromatin organisation, downregulation of chromatin organization, downregulation of establishment or maintenance of chromatin architecture, negative regulation of chromatin assembly/disassembly, negative regulation of chromatin organisation, negative regulation of establishment or maintenance of chromatin architecture, inhibition of chromatin assembly or disassembly, inhibition of chromatin organisation, inhibition of chromatin organization, inhibition of establishment or maintenance of chromatin architecture, down regulation of chromatin assembly or disassembly, down-regulation of chromatin assembly or disassembly, downregulation of chromatin assembly or disassembly, negative regulation of chromatin assembly or disassembly, negative regulation of chromatin modification Definition: Any process that stops, prevents or reduces the frequency, rate or extent of chromatin organization.